{
  "gene_symbol": "OR51C1",
  "gene": "UniProtKB:A0A3B3IT45",
  "term_label": "plasma membrane",
  "term_id": "GO:0005886",
  "gene_name": "Olfactory receptor"
}